{
  "term_id": "GO:0005588",
  "gene_symbol": "COL5A1",
  "gene_name": "Collagen alpha-1(V) chain",
  "term_label": "collagen type V trimer",
  "gene": "UniProtKB:P20908"
}